{
  "gene_symbol": "MT-ATP8",
  "gene_name": "ATP synthase protein 8",
  "gene": "UniProtKB:P03928",
  "term_id": "GO:0042776",
  "term_label": "proton motive force-driven mitochondrial ATP synthesis"
}